{
  "gene_name": "Condensin-2 complex subunit D3",
  "gene": "UniProtKB:P42695",
  "gene_symbol": "NCAPD3",
  "term_id": "GO:0007076",
  "term_label": "mitotic chromosome condensation"
}